{
  "gene_name": "Dedicator of cytokinesis protein 3",
  "term_label": "plasma membrane",
  "term_id": "GO:0005886",
  "gene": "UniProtKB:Q8IZD9",
  "gene_symbol": "DOCK3"
}